{
  "gene_name": "Mitochondrial tRNA methylthiotransferase CDK5RAP1",
  "term_label": "mitochondrion",
  "gene_symbol": "CDK5RAP1",
  "gene": "UniProtKB:Q96SZ6",
  "term_id": "GO:0005739"
}